{
  "term_label": "Unknown cellular component",
  "gene_name": "Putative uncharacterized protein SCP2D1-AS1",
  "term_id": "UNKNOWN:0003",
  "gene": "UniProtKB:Q9BR46",
  "gene_symbol": "SCP2D1-AS1"
}